{
  "term_id": "GO:0036505",
  "gene": "UniProtKB:O15354",
  "gene_name": "Prosaposin receptor GPR37",
  "gene_symbol": "GPR37",
  "term_label": "prosaposin receptor activity"
}